{
  "term_label": "toll-like receptor 4 signaling pathway",
  "gene": "UniProtKB:Q9BQ95",
  "term_id": "GO:0034142",
  "gene_name": "Evolutionarily conserved signaling intermediate in Toll pathway, mitochondrial",
  "gene_symbol": "ECSIT"
}